positive regulation of natural killer cell differentiation involved in immune response [GO:0032828] (BP) Note: Note that immunologists typically use the word 'development' to refer to cells of B or T cell lineages undergoing the process that GO describes as 'cell differentiation'. Also known as: activation of natural killer cell differentiation during immune response, stimulation of natural killer cell differentiation during immune response, positive regulation of NK cell differentiation during immune response, positive regulation of natural killer cell development involved in immune response, positive regulation of natural killer cell differentiation during immune response, up regulation of natural killer cell differentiation during immune response, up-regulation of natural killer cell differentiation during immune response, upregulation of natural killer cell differentiation during immune response Relationships: is a type of positive regulation of immune effector process [GO:0002699]; is a type of positive regulation of natural killer cell differentiation [GO:0032825]; is a type of regulation of natural killer cell differentiation involved in immune response [GO:0032826]; is a type of positive regulation of immune response [GO:0050778]; RO_0002213 natural killer cell differentiation involved in immune response [GO:0002325] Sources: GOC:mah Definition: Any process that activates or increases the frequency, rate or extent of natural killer cell differentiation as part of an immune response.